{
  "gene_symbol": "SMARCC2",
  "term_id": "GO:0071564",
  "term_label": "npBAF complex",
  "gene_name": "SWI_SNF complex subunit SMARCC2",
  "gene": "UniProtKB:Q8TAQ2"
}